{
  "term_label": "structural constituent of ribosome",
  "term_id": "GO:0003735",
  "gene_name": "Large ribosomal subunit protein bL19m",
  "gene_symbol": "MRPL19",
  "gene": "UniProtKB:P49406"
}